{
  "gene": "UniProtKB:Q9UGH3",
  "gene_symbol": "SLC23A2",
  "term_label": "L-ascorbic acid transmembrane transport",
  "gene_name": "Solute carrier family 23 member 2",
  "term_id": "GO:0015882"
}